{
  "gene_name": "Vesicle transport protein USE1",
  "term_id": "GO:0005783",
  "term_label": "endoplasmic reticulum",
  "gene": "UniProtKB:Q9NZ43",
  "gene_symbol": "USE1"
}